{
  "gene": "UniProtKB:Q9UJ99",
  "term_label": "adherens junction organization",
  "gene_name": "Cadherin-22",
  "term_id": "GO:0034332",
  "gene_symbol": "CDH22"
}